maltose transporting porin activity [GO:0015481] (molecular function) Sources: GOC:mtg_transport Also known as: maltoporin Relationships: is_a maltose transmembrane transporter activity [GO:0005363]; is a type of porin activity [GO:0015288] Definition: Enables the transfer of maltose from one side of a membrane to the other. Maltose is the disaccharide 4-O-alpha-D-glucopyranosyl-D-glucopyranose, an intermediate in the enzymatic breakdown of glycogen and starch. This transporter is a porin so enables the energy independent passage of substances, sized less than 1000 Da, across a membrane. The transmembrane portions of porins consist exclusively of beta-strands which form a beta-barrel. They are found in the outer membranes of Gram-negative bacteria, mitochondria, plastids and possibly acid-fast Gram-positive bacteria.